negative regulation of developmental growth [GO:0048640] (biological process) Relationships: is a type of negative regulation of growth [GO:0045926]; is a type of regulation of developmental growth [GO:0048638]; is a type of negative regulation of developmental process [GO:0051093]; negatively regulates developmental growth [GO:0048589] Definition: Any process that stops, prevents, or reduces the frequency, rate or extent of developmental growth. Also known as: down regulation of developmental growth, down-regulation of developmental growth, downregulation of developmental growth, inhibition of developmental growth Sources: GOC:go_curators Subtypes: GO:0030517, negative regulation of multicellular organism growth [GO:0040015], negative regulation of skeletal muscle tissue regeneration [GO:0043417], negative regulation of imaginal disc growth [GO:0045571], GO:0045886, GO:0046621, negative regulation of skeletal muscle tissue growth [GO:0048632], negative regulation of collateral sprouting [GO:0048671], negative regulation of sprouting of injured axon [GO:0048688], negative regulation of unidimensional cell growth [GO:0051511], GO:0061112, negative regulation of branch elongation involved in ureteric bud branching [GO:0072096], GO:1901233, negative regulation of root hair elongation [GO:1902891], negative regulation of chondrocyte hypertrophy [GO:1903042], negative regulation of dendrite extension [GO:1903860], negative regulation of epithelium regeneration [GO:1905042], negative regulation of cardiac muscle tissue regeneration [GO:1905179], negative regulation of developmental vegetative growth [GO:1905614]